{
  "term_id": "UNKNOWN:0002",
  "gene": "UniProtKB:Q9UBP9",
  "gene_symbol": "GULP1",
  "term_label": "Unknown biological process",
  "gene_name": "PTB domain-containing engulfment adapter protein 1"
}